{
  "term_label": "centrosome",
  "gene_name": "Rho guanine nucleotide exchange factor 10",
  "term_id": "GO:0005813",
  "gene": "UniProtKB:O15013",
  "gene_symbol": "ARHGEF10"
}